{
  "term_label": "Unknown cellular component",
  "gene_symbol": "IGHV1OR21-1",
  "term_id": "UNKNOWN:0003",
  "gene_name": "Immunoglobulin heavy variable 1_OR21-1 (non-functional) (Fragment)",
  "gene": "UniProtKB:A0A087WYE8"
}